4-(hydroxymethyl)benzenesulfonate dehydrogenase activity [GO:0018462] (molecular function) Definition: Catalysis of the reaction: 4-(hydroxymethyl)benzenesulfonate + NAD+ = 4-formylbenzenesulfonate + H+ + NADH. Also known as: 4-(hydroxymethyl)benzenesulphonate dehydrogenase activity, 4-sulfobenzyl alcohol dehydrogenase activity, 4-(hydroxymethyl)benzenesulfonate:NAD+ oxidoreductase activity Sources: EC:1.1.1.257, RHEA:24412 Relationships: is a type of GO:0016616